{
  "term_id": "GO:0005829",
  "gene_symbol": "CERT1",
  "gene": "UniProtKB:Q9Y5P4",
  "gene_name": "Ceramide transfer protein",
  "term_label": "cytosol"
}